{
  "gene_name": "Golgin subfamily A member 6-like protein 9",
  "term_id": "UNKNOWN:0002",
  "gene": "UniProtKB:A6NEM1",
  "term_label": "Unknown biological process",
  "gene_symbol": "GOLGA6L9"
}